{
  "term_label": "extracellular space",
  "gene_name": "Agouti-signaling protein",
  "term_id": "GO:0005615",
  "gene_symbol": "ASIP",
  "gene": "UniProtKB:P42127"
}